{
  "gene": "UniProtKB:P02489",
  "gene_name": "Alpha-crystallin A chain",
  "term_label": "response to heat",
  "gene_symbol": "CRYAA",
  "term_id": "GO:0009408"
}